{
  "term_id": "GO:0022627",
  "gene": "UniProtKB:P62857",
  "term_label": "cytosolic small ribosomal subunit",
  "gene_name": "Small ribosomal subunit protein eS28",
  "gene_symbol": "RPS28"
}